17-methylnonadec-1-ene biosynthetic process [GO:1900883] (biological process) Relationships: is a type of GO:0043450; is a type of 17-methylnonadec-1-ene metabolic process [GO:1900882] Definition: The chemical reactions and pathways resulting in the formation of 17-methylnonadec-1-ene. Sources: GOC:TermGenie, GOC:mengo_curators Regulation: regulated by regulation of 17-methylnonadec-1-ene biosynthetic process [GO:1900956]; negatively regulated by GO:1900957; positively regulated by positive regulation of 17-methylnonadec-1-ene biosynthetic process [GO:1900958] Also known as: 17-methylnonadec-1-ene anabolism, 17-methylnonadec-1-ene biosynthesis, 17-methylnonadec-1-ene formation, 17-methylnonadec-1-ene synthesis